{
  "gene_symbol": "AADACL2",
  "term_label": "Unknown cellular component",
  "gene_name": "Arylacetamide deacetylase-like 2",
  "gene": "UniProtKB:Q6P093",
  "term_id": "UNKNOWN:0003"
}